{
  "gene": "UniProtKB:P42766",
  "gene_name": "Large ribosomal subunit protein uL29",
  "term_id": "GO:0003735",
  "gene_symbol": "RPL35",
  "term_label": "structural constituent of ribosome"
}